{
  "gene": "UniProtKB:P29376",
  "term_id": "GO:0007169",
  "gene_symbol": "LTK",
  "gene_name": "Leukocyte tyrosine kinase receptor",
  "term_label": "cell surface receptor protein tyrosine kinase signaling pathway"
}